5' overhang single-stranded DNA endodeoxyribonuclease activity [GO:1990601] (molecular function) Definition: Catalysis of the hydrolysis of ester linkages within 5' overhang single-stranded deoxyribonucleic acid by creating internal breaks. Relationships: is a type of single-stranded DNA endodeoxyribonuclease activity [GO:0000014] References: PMID:25203555